{
  "term_id": "UNKNOWN:0001",
  "term_label": "Unknown molecular function",
  "gene_name": "Zinc finger protein 157",
  "gene": "UniProtKB:P51786",
  "gene_symbol": "ZNF157"
}